{
  "gene_symbol": "FGF22",
  "term_label": "regulation of cell migration",
  "term_id": "GO:0030334",
  "gene_name": "Fibroblast growth factor 22",
  "gene": "UniProtKB:Q9HCT0"
}